perforation plate [GO:1990073] (cellular component) Note: Part of a vessel member (PO:0002003). May be simple, with one perforation, or multiperforate, with more than one perforation. Perforation plates are usually on the end walls of a cell, but may also be on the side walls. Relationships: is_a GO:0110165; is part of GO:0005618 Definition: A cell wall part that is the part of a wall of a vessel member and bears one or more openings (perforations). Sources: GOC:PO_curators, ISBN:0471245194